diacylglycerol catabolic process [GO:0046340] (biological process) Definition: The chemical reactions and pathways resulting in the breakdown of diacylglycerol, a glyceride in which any two of the R groups (positions not specified) are acyl groups while the remaining R group can be either H or an alkyl group. References: PMID:11717312 Relationships: is a type of diacylglycerol metabolic process [GO:0046339]; is_a acylglycerol catabolic process [GO:0046464] Also known as: diacylglycerol breakdown, diacylglycerol catabolism, diacylglycerol degradation, diglyceride catabolism